{
  "gene_symbol": "SPHK2",
  "gene": "UniProtKB:Q9NRA0",
  "gene_name": "Sphingosine kinase 2",
  "term_id": "GO:0005886",
  "term_label": "plasma membrane"
}